regulation of epidermal cell differentiation [GO:0045604] (biological process) Relationships: is a type of regulation of epithelial cell differentiation [GO:0030856]; is_a regulation of epidermis development [GO:0045682]; regulates epidermal cell differentiation [GO:0009913] Subtypes: negative regulation of epidermal cell differentiation [GO:0045605], positive regulation of epidermal cell differentiation [GO:0045606], regulation of inner ear auditory receptor cell differentiation [GO:0045607], regulation of keratinocyte differentiation [GO:0045616] Definition: Any process that modulates the frequency, rate or extent of epidermal cell differentiation. Sources: GOC:go_curators Also known as: regulation of hypodermal cell differentiation